{
  "term_id": "GO:0002767",
  "gene": "UniProtKB:P43629",
  "term_label": "immune response-inhibiting cell surface receptor signaling pathway",
  "gene_name": "Killer cell immunoglobulin-like receptor 3DL1",
  "gene_symbol": "KIR3DL1"
}